{
  "term_id": "GO:0022625",
  "gene": "UniProtKB:P62913",
  "gene_symbol": "RPL11",
  "term_label": "cytosolic large ribosomal subunit",
  "gene_name": "Large ribosomal subunit protein uL5"
}